SUMO transferase activity [GO:0019789] (molecular function) Also known as: SMT3 conjugating enzyme, SUMO conjugating enzyme activity References: PMID:11031248, PMID:11265250 Sources: GOC:rn Definition: Catalysis of the transfer of SUMO from one protein to another via the reaction X-SUMO + Y = Y-SUMO + X, where both X-SUMO and Y-SUMO are covalent linkages. Subtypes: SUMO conjugating enzyme activity [GO:0061656], SUMO ligase activity [GO:0061665] Relationships: is a type of ubiquitin-like protein transferase activity [GO:0019787]